{
  "term_label": "Unknown molecular function",
  "gene": "UniProtKB:Q8N268",
  "term_id": "UNKNOWN:0001",
  "gene_symbol": "LINC02910",
  "gene_name": "Putative uncharacterized protein encoded by LINC02910"
}